{
  "term_label": "Golgi apparatus",
  "gene_symbol": "VTI1B",
  "gene": "UniProtKB:Q9UEU0",
  "term_id": "GO:0005794",
  "gene_name": "Vesicle transport through interaction with t-SNAREs homolog 1B"
}